sporangiospore formation [GO:0034300] (biological process) Definition: The process in which sporangiospores, a type of asexual spore found in fungi, are formed. Sporangiospores are formed within sac-like structure, the sporangium, following the division of the cytoplasm. References: PMID:32839172 Sources: GOC:ds, GOC:mah Relationships: is a type of asexual sporulation resulting in formation of a cellular spore [GO:0043936] Subtypes: GO:0075239, aplanospore formation [GO:0075289] Regulation: regulated by regulation of sporangiospore formation [GO:0075286]; positively regulated by positive regulation of sporangiospore formation [GO:0075287]; negatively regulated by negative regulation of sporangiospore formation [GO:0075288]